{
  "gene": "UniProtKB:P0DKL9",
  "gene_name": "ARL14 effector protein-like",
  "term_label": "Unknown cellular component",
  "term_id": "UNKNOWN:0003",
  "gene_symbol": "ARL14EPL"
}